{
  "term_label": "trehalose catabolic process",
  "gene_name": "Trehalase",
  "gene": "UniProtKB:O43280",
  "term_id": "GO:0005993",
  "gene_symbol": "TREH"
}